calpain complex [GO:0110158] (cellular component) Relationships: is a type of GO:0008303; is part of cytoplasm [GO:0005737] Definition: A calcium-dependent protease complex that processes its substrate by limited proteolysis rather than degrading it. In some cases limited proteolysis is required for the activation of its substrate. References: PMID:10639123 Sources: GOC:bhm Also known as: M-calpain, mu-calpain